L-arabinokinase activity [GO:0009702] (molecular function) Relationships: is a type of phosphotransferase activity, alcohol group as acceptor [GO:0016773]; is a type of carbohydrate kinase activity [GO:0019200] Sources: EC:2.7.1.46, RHEA:20153 Also known as: ATP:L-arabinose 1-phosphotransferase activity, L-arabinokinase (phosphorylating) Definition: Catalysis of the reaction: L-arabinose + ATP = beta-L-arabinose 1-phosphate + ADP + 2 H+.